{
  "term_id": "GO:0048471",
  "gene_name": "Heat shock protein HSP 90-beta",
  "gene": "UniProtKB:P08238",
  "gene_symbol": "HSP90AB1",
  "term_label": "perinuclear region of cytoplasm"
}